cobalamin binding [GO:0031419] (molecular function) Definition: Binding to cobalamin (vitamin B12), a water-soluble vitamin characterized by possession of a corrin nucleus containing a cobalt atom. Also known as: vitamin B12 binding Sources: GOC:mah Relationships: is_a vitamin binding [GO:0019842]; is a type of tetrapyrrole binding [GO:0046906]; is a type of heterocyclic compound binding [GO:1901363]